Cvt complex [GO:0034270] (cellular component) References: PMID:15659643 Sources: GOC:rb Definition: A protein complex that is involved in the Cvt pathway. In budding yeast, the Cvt complex consists of multimers of preApe1p. Relationships: is a type of GO:0032991; is part of cytoplasm [GO:0005737] Also known as: cytoplasm to vacuole targeting complex, cytoplasm-to-vacuole targeting complex